phospholipid binding [GO:0005543] (molecular function) Subtypes: phosphatidylserine binding [GO:0001786], GO:0005544, phosphatidylethanolamine binding [GO:0008429], phosphatidylcholine binding [GO:0031210], phosphatidylinositol binding [GO:0035091], GO:0035727, phosphatidic acid binding [GO:0070300], GO:1901611, ceramide 1-phosphate binding [GO:1902387] Relationships: is a type of lipid binding [GO:0008289] Sources: ISBN:0198506732 Definition: Binding to a phospholipid, a class of lipids containing phosphoric acid as a mono- or diester.